{
  "gene_name": "PCI domain-containing protein 2",
  "gene_symbol": "PCID2",
  "gene": "UniProtKB:Q5JVF3",
  "term_label": "poly(A)+ mRNA export from nucleus",
  "term_id": "GO:0016973"
}